{
  "gene_name": "Nuclear distribution protein nudE-like 1",
  "term_label": "centrosome",
  "gene": "UniProtKB:Q9GZM8",
  "term_id": "GO:0005813",
  "gene_symbol": "NDEL1"
}